alkanal monooxygenase (FMN-linked) activity [GO:0047646] (molecular function) Sources: EC:1.14.14.3, MetaCyc:ALKANAL-MONOOXYGENASE-FMN-LINKED-RXN Relationships: is a type of oxidoreductase activity, acting on paired donors, with incorporation or reduction of molecular oxygen, reduced flavin or flavoprotein as one donor, and incorporation of one atom of oxygen [GO:0016712] Definition: Catalysis of the reaction: R-CHO + reduced FMN + O2 = R-COOH + FMN + H2O + light. Also known as: aldehyde monooxygenase activity, alkanal,reduced-FMN:oxygen oxidoreductase (1-hydroxylating, luminescing), bacterial luciferase activity, vibrio fischeri luciferase activity